{
  "gene": "UniProtKB:P29558",
  "gene_symbol": "RBMS1",
  "term_id": "UNKNOWN:0002",
  "term_label": "Unknown biological process",
  "gene_name": "RNA-binding motif, single-stranded-interacting protein 1"
}